{
  "gene_symbol": "DUSP4",
  "term_id": "GO:0001706",
  "gene": "UniProtKB:Q13115",
  "gene_name": "Dual specificity protein phosphatase 4",
  "term_label": "endoderm formation"
}